{
  "gene_symbol": "PATE2",
  "term_id": "UNKNOWN:0002",
  "gene_name": "Prostate and testis expressed protein 2",
  "gene": "UniProtKB:Q6UY27",
  "term_label": "Unknown biological process"
}